adrenal chromaffin cell differentiation [GO:0061104] (BP) Sources: GOC:dph Relationships: is a type of glandular epithelial cell differentiation [GO:0002067]; is a type of neuroendocrine cell differentiation [GO:0061101]; is part of adrenal gland development [GO:0030325] Definition: The process in which a relatively unspecialized cell acquires specialized structural and/or functional features of an adrenal chromaffin cell. An adrenal chromaffin cell is a neuroendocrine cell that stores epinephrine secretory vesicles.